positive regulation of p38MAPK cascade [GO:1900745] (biological process) Definition: Any process that activates or increases the frequency, rate or extent of p38MAPK cascade. Also known as: activation of p38 MAPK cascade, activation of p38 cascade, positive regulation of p38 MAPK cascade, positive regulation of p38 cascade, up regulation of p38 MAPK cascade, up regulation of p38 cascade, up regulation of p38MAPK cascade, up-regulation of p38 MAPK cascade, up-regulation of p38 cascade, up-regulation of p38MAPK cascade, upregulation of p38 MAPK cascade, upregulation of p38 cascade, upregulation of p38MAPK cascade, activation of p38MAPK cascade, positive regulation of osmosensory signaling MAPK cascade Sources: GOC:TermGenie Relationships: is a type of positive regulation of MAPK cascade [GO:0043410]; is a type of GO:1900744; positively regulates p38MAPK cascade [GO:0038066]